{
  "gene_name": "Dual specificity protein phosphatase 8",
  "gene": "UniProtKB:Q13202",
  "term_id": "GO:0008330",
  "gene_symbol": "DUSP8",
  "term_label": "protein tyrosine/threonine phosphatase activity"
}